{
  "gene_name": "Exocyst complex component 2",
  "gene_symbol": "EXOC2",
  "gene": "UniProtKB:Q96KP1",
  "term_id": "GO:0006893",
  "term_label": "Golgi to plasma membrane transport"
}